{
  "term_label": "syntaxin-1 binding",
  "term_id": "GO:0017075",
  "gene": "UniProtKB:Q15836",
  "gene_symbol": "VAMP3",
  "gene_name": "Vesicle-associated membrane protein 3"
}